{
  "term_label": "regulation of cellular pH",
  "gene_symbol": "ATP6AP1",
  "gene_name": "V-type proton ATPase subunit S1",
  "gene": "UniProtKB:Q15904",
  "term_id": "GO:0030641"
}